{
  "gene_name": "Inactive peptidyl-prolyl cis-trans isomerase FKBP6",
  "term_label": "piRNA processing",
  "term_id": "GO:0034587",
  "gene_symbol": "FKBP6",
  "gene": "UniProtKB:O75344"
}